hercynylcysteine sulfoxide synthase activity [GO:0061686] (molecular function) Also known as: hercynylcysteine S-oxide synthase, hercynylcysteine sulfoxide synthase Definition: Catalysis of the reaction: L-cysteine + N-alpha,N-alpha,N-alpha-trimethyl-L-histidine (hercynine) + O2 = hercynylcysteine sulfoxide + H2O. References: PMID:24828577, PMID:4276459 Sources: GOC:dph, RHEA:42704 Relationships: is a type of oxidoreductase activity, acting on X-H and Y-H to form an X-Y bond, with oxygen as acceptor [GO:0046993]; is part of ergothioneine biosynthesis from histidine via hercynylcysteine sulfoxide synthase [GO:0140479]